plant ovule morphogenesis [GO:0048482] (biological process) Relationships: is a type of developmental process involved in reproduction [GO:0003006]; is a type of GO:0090698; is a type of GO:1905392; is part of carpel morphogenesis [GO:0048445]; is part of plant ovule development [GO:0048481] Sources: GOC:tb Definition: The process in which the anatomical structures of the ovule are generated and organized. The ovule is the structure in seed plants enclosing the female gametophyte, and is composed of the nucellus, one or two integuments, and the funiculus; it develops into the seed.